{
  "gene": "UniProtKB:O14646",
  "gene_name": "Chromodomain-helicase-DNA-binding protein 1",
  "term_label": "ATP-dependent chromatin remodeler activity",
  "term_id": "GO:0140658",
  "gene_symbol": "CHD1"
}